bioadhesive activity [GO:0140073] (molecular function) Definition: A structural molecule ativity that mediates an organism's attachment to an environmental substrate via stable, non-selective binding by a protein to an external surface. Examples includes proteins used by insects to anchor pupae to surfaces. Relationships: is a type of GO:0005198 References: PMID:39370426